{
  "term_id": "GO:0045109",
  "term_label": "intermediate filament organization",
  "gene_symbol": "KRT2",
  "gene_name": "Keratin, type II cytoskeletal 2 epidermal",
  "gene": "UniProtKB:P35908"
}